{
  "gene_name": "Zinc finger protein 398",
  "term_id": "GO:0000977",
  "gene_symbol": "ZNF398",
  "term_label": "RNA polymerase II transcription regulatory region sequence-specific DNA binding",
  "gene": "UniProtKB:Q8TD17"
}